{
  "gene": "UniProtKB:Q96PR1",
  "term_label": "dendrite membrane",
  "gene_name": "Potassium voltage-gated channel subfamily C member 2",
  "gene_symbol": "KCNC2",
  "term_id": "GO:0032590"
}